regulation of leukocyte cell-cell adhesion [GO:1903037] (biological process) Subtypes: regulation of monocyte aggregation [GO:1900623], GO:1903038, positive regulation of leukocyte cell-cell adhesion [GO:1903039], regulation of leukocyte adhesion to vascular endothelial cell [GO:1904994], regulation of thymocyte aggregation [GO:2000398], regulation of neutrophil aggregation [GO:2000428], regulation of T cell costimulation [GO:2000523] Relationships: is a type of regulation of cell-cell adhesion [GO:0022407]; regulates GO:0007159 Definition: Any process that modulates the frequency, rate or extent of leukocyte cell-cell adhesion. References: PMID:21106532 Sources: GOC:BHF, GOC:TermGenie, GOC:rl, GO_REF:0000058 Also known as: regulation of leukocyte adhesion, regulation of leukocyte cell adhesion Note: Exogenous expression of ASS1 or NOS3 in HUVECs enhances NO production and inhibits monocyte adhesion